cardiac glial cell fate commitment [GO:0060953] (BP) Subtypes: neural crest-derived cardiac glial cell fate commitment [GO:0060955] Definition: The commitment of cells to cardiac glial cell fates and their capacity to differentiate into cardiac glial cells. Relationships: is a type of glial cell fate commitment [GO:0021781]; is_a cardiac cell fate commitment [GO:0060911]; is part of cardiac glial cell differentiation [GO:0060950] Sources: GOC:mtg_heart